{
  "term_label": "plasma membrane",
  "gene": "UniProtKB:Q99571",
  "term_id": "GO:0005886",
  "gene_name": "P2X purinoceptor 4",
  "gene_symbol": "P2RX4"
}